{
  "term_id": "GO:0031514",
  "term_label": "motile cilium",
  "gene_symbol": "ROPN1B",
  "gene": "UniProtKB:Q9BZX4",
  "gene_name": "Ropporin-1B"
}